{
  "term_label": "cytosol",
  "gene": "UniProtKB:Q92748",
  "gene_name": "Thyroid hormone-inducible hepatic protein",
  "term_id": "GO:0005829",
  "gene_symbol": "THRSP"
}